{
  "term_id": "GO:0006357",
  "gene": "UniProtKB:Q6ZNG0",
  "term_label": "regulation of transcription by RNA polymerase II",
  "gene_name": "Zinc finger protein 620",
  "gene_symbol": "ZNF620"
}